{
  "gene_symbol": "ZNF606",
  "gene_name": "Zinc finger protein 606",
  "term_id": "GO:0005634",
  "term_label": "nucleus",
  "gene": "UniProtKB:Q8WXB4"
}